{
  "term_id": "GO:0005886",
  "gene_symbol": "TTC7A",
  "gene_name": "Tetratricopeptide repeat protein 7A",
  "term_label": "plasma membrane",
  "gene": "UniProtKB:Q9ULT0"
}